{
  "term_id": "GO:0008289",
  "gene_name": "Apolipoprotein L4",
  "term_label": "lipid binding",
  "gene_symbol": "APOL4",
  "gene": "UniProtKB:Q9BPW4"
}